isotype switching to IgE isotypes [GO:0048289] (biological process) Subtypes: GO:0035708 Regulation: RO_0002211 by regulation of isotype switching to IgE isotypes [GO:0048293]; negatively regulated by GO:0048294; positively regulated by positive regulation of isotype switching to IgE isotypes [GO:0048295] Definition: The switching of activated B cells from IgM biosynthesis to IgE biosynthesis, accomplished through a recombination process involving an intrachromosomal deletion between switch regions that reside 5' of the IgM and IgE constant region gene segments in the immunoglobulin heavy chain locus. Also known as: class switch recombination to IgE isotypes, class switching to IgE isotypes, isotype switch recombination to IgE isotypes References: PMID:12370374, PMID:2113175, PMID:9186655 Sources: ISBN:0781735149 Relationships: is a type of isotype switching [GO:0045190]